negative regulation of T cell extravasation [GO:2000408] (biological process) Sources: GOC:BHF, GOC:mah Relationships: is a type of negative regulation of cellular extravasation [GO:0002692]; is a type of GO:2000405; is a type of regulation of T cell extravasation [GO:2000407]; negatively regulates T cell extravasation [GO:0072683] Subtypes: negative regulation of CD8-positive, alpha-beta T cell extravasation [GO:2000450] Also known as: negative regulation of T lymphocyte extravasation, negative regulation of T-cell extravasation, negative regulation of T-lymphocyte extravasation Definition: Any process that stops, prevents or reduces the frequency, rate or extent of T cell extravasation.